{
  "term_id": "UNKNOWN:0001",
  "gene_name": "Pleckstrin homology domain-containing family M member 1",
  "term_label": "Unknown molecular function",
  "gene_symbol": "PLEKHM1",
  "gene": "UniProtKB:Q9Y4G2"
}